growth hormone-releasing hormone receptor activity [GO:0016520] (molecular function) Relationships: is a type of GO:0004930 Definition: Combining with growth hormone-releasing hormone to initiate a change in cell activity. References: PMID:12529933